{
  "gene_symbol": "ITGA5",
  "gene_name": "Integrin alpha-5",
  "gene": "UniProtKB:P08648",
  "term_id": "GO:0098609",
  "term_label": "cell-cell adhesion"
}